{
  "gene_symbol": "PGP",
  "gene_name": "Glycerol-3-phosphate phosphatase",
  "gene": "UniProtKB:A6NDG6",
  "term_id": "GO:0005737",
  "term_label": "cytoplasm"
}